odontoblast differentiation [GO:0071895] (biological process) References: PMID:20425127 Sources: GOC:sl Relationships: is a type of GO:0060563 Regulation: regulated by regulation of odontoblast differentiation [GO:1901329]; negatively regulated by negative regulation of odontoblast differentiation [GO:1901330]; positively regulated by positive regulation of odontoblast differentiation [GO:1901331] Definition: The process in which a relatively unspecialized cell of neural crest origin acquires the specialized features of an odontoblast, a cell on the outer surface of the dental pulp whose biological function is the creation of dentin.